H-NS-Hha complex [GO:0097495] (cellular component) Definition: A trimeric protein complex made up of an H-NS homodimer and an Hha monomer. In Enterobacteriaceae, this complex negatively regulates transcription of a range of genes. References: PMID:21600204 Sources: GOC:bhm Relationships: is a type of protein-containing complex [GO:0032991]; is part of GO:0005829; has part H-NS complex [GO:1990121]